{
  "gene_symbol": "VGLL3",
  "gene_name": "Transcription cofactor vestigial-like protein 3",
  "term_id": "UNKNOWN:0001",
  "gene": "UniProtKB:A8MV65",
  "term_label": "Unknown molecular function"
}